{
  "term_label": "Unknown biological process",
  "term_id": "UNKNOWN:0002",
  "gene_symbol": "FAM131B",
  "gene": "UniProtKB:Q86XD5",
  "gene_name": "Protein FAM131B"
}